{
  "gene": "UniProtKB:Q9UKG1",
  "term_id": "GO:0023052",
  "gene_name": "DCC-interacting protein 13-alpha",
  "term_label": "signaling",
  "gene_symbol": "APPL1"
}